{
  "term_id": "GO:0000380",
  "gene_name": "Probable ATP-dependent RNA helicase DDX17",
  "gene": "UniProtKB:Q92841",
  "gene_symbol": "DDX17",
  "term_label": "alternative mRNA splicing, via spliceosome"
}